{
  "gene": "UniProtKB:P02675",
  "gene_name": "Fibrinogen beta chain",
  "gene_symbol": "FGB",
  "term_label": "extracellular space",
  "term_id": "GO:0005615"
}